{
  "term_label": "keratin filament",
  "gene_name": "Keratin, type II cytoskeletal 75",
  "gene_symbol": "KRT75",
  "term_id": "GO:0045095",
  "gene": "UniProtKB:O95678"
}